{
  "gene_symbol": "KRT77",
  "term_id": "GO:0030280",
  "term_label": "structural constituent of skin epidermis",
  "gene_name": "Keratin, type II cytoskeletal 1b",
  "gene": "UniProtKB:Q7Z794"
}